cell communication [GO:0007154] (biological process) Subtypes: response to pheromone regulating conjugation with mutual genetic exchange [GO:0000756], cell-cell signaling [GO:0007267], axon target recognition [GO:0007412], sex determination, somatic-gonadal interaction [GO:0007543], pollen-pistil interaction [GO:0009875], cell communication by chemical coupling [GO:0010643], cell communication by electrical coupling [GO:0010644], motogenic signaling initiating cell movement in cerebral cortex [GO:0021807], motogenic signaling involved in postnatal olfactory bulb interneuron migration [GO:0021837], motogenic signaling involved in interneuron migration from the subpallium to the cortex [GO:0021838], extracellular matrix-cell signaling [GO:0035426], GO:0086065 Sources: GOC:mah Definition: Any process that mediates interactions between a cell and its surroundings. Encompasses interactions such as signaling or attachment between one cell and another cell, between a cell and an extracellular matrix, or between a cell and any other aspect of its environment. Relationships: is a type of GO:0009987 Regulation: regulated by regulation of cell communication [GO:0010646]; RO_0002213 by positive regulation of cell communication [GO:0010647]; negatively regulated by negative regulation of cell communication [GO:0010648]